{
  "term_label": "Unknown molecular function",
  "term_id": "UNKNOWN:0001",
  "gene_symbol": "AMIGO3",
  "gene_name": "Amphoterin-induced protein 3",
  "gene": "UniProtKB:Q86WK7"
}